{
  "gene_name": "Ganglioside GM2 activator",
  "gene": "UniProtKB:P17900",
  "term_id": "GO:0005319",
  "term_label": "lipid transporter activity",
  "gene_symbol": "GM2A"
}